{
  "term_label": "Unknown cellular component",
  "gene": "UniProtKB:Q8IZP2",
  "term_id": "UNKNOWN:0003",
  "gene_symbol": "ST13P4",
  "gene_name": "Putative protein FAM10A4"
}